{
  "term_id": "UNKNOWN:0003",
  "term_label": "Unknown cellular component",
  "gene_name": "Solute carrier family 22 member 2",
  "gene": "UniProtKB:O15244",
  "gene_symbol": "SLC22A2"
}